gastrulation [GO:0007369] (biological process) Relationships: is a type of embryonic morphogenesis [GO:0048598]; has part ectoderm formation [GO:0001705]; has part endoderm formation [GO:0001706]; has part mesoderm formation [GO:0001707] Definition: A complex and coordinated series of cellular movements that occurs at the end of cleavage during embryonic development of most animals. The details of gastrulation vary from species to species, but usually result in the formation of the three primary germ layers, ectoderm, mesoderm and endoderm. Regulation: regulated by GO:0010470; negatively regulated by negative regulation of gastrulation [GO:2000542]; positively regulated by positive regulation of gastrulation [GO:2000543] Sources: GOC:curators, ISBN:9780878933846 Subtypes: gastrulation with mouth forming second [GO:0001702], GO:0001703